{
  "term_label": "DNA-binding transcription factor activity, RNA polymerase II-specific",
  "gene": "UniProtKB:Q9H7R5",
  "term_id": "GO:0000981",
  "gene_symbol": "ZNF665",
  "gene_name": "Zinc finger protein 665"
}